cuneatus tract morphogenesis [GO:0021959] (biological process) References: PMID:12867698 Sources: GOC:cls, GOC:dgh, GOC:dph, GOC:jid, GO_REF:0000021 Definition: Generation of a long process of a CNS neuron, that carries efferent (outgoing) action potentials from the cell body in the dorsal root ganglion towards target cells in the medulla. This axonal process is a member of those that make up the cuneatus tract, a group of axons that are from neurons involved in proprioception from the upper trunk and upper limb. Relationships: is a type of central nervous system projection neuron axonogenesis [GO:0021952] Also known as: tract of Burdach morphogenesis